{
  "gene": "UniProtKB:H3BSY2",
  "term_id": "UNKNOWN:0001",
  "term_label": "Unknown molecular function",
  "gene_name": "Golgin subfamily A member 8M",
  "gene_symbol": "GOLGA8M"
}